{
  "gene": "UniProtKB:P35968",
  "gene_name": "Vascular endothelial growth factor receptor 2",
  "term_label": "angiogenesis",
  "gene_symbol": "KDR",
  "term_id": "GO:0001525"
}